transcription factor TFIIH holo complex [GO:0005675] (cellular component) Definition: A complex that is capable of kinase activity directed towards the C-terminal Domain (CTD) of the largest subunit of RNA polymerase II and is essential for initiation at RNA polymerase II promoters in vitro. It is composed of the core TFIIH complex and the TFIIK complex. Relationships: is a type of nuclear cyclin-dependent protein kinase holoenzyme complex [GO:0019908]; is a type of GO:0032806; is a type of RNA polymerase II transcription regulator complex [GO:0090575]; is part of RNA polymerase II, holoenzyme [GO:0016591]; has part transcription factor TFIIH core complex [GO:0000439] References: PMID:14500720, PMID:22308316, PMID:22572993, PMID:7813015 Sources: GOC:ew, GOC:krc Also known as: CDK-activating kinase, cyclin-dependent protein kinase activating kinase holoenzyme complex, holo TFIIH complex, CAK complex